{
  "gene_symbol": "KLK14",
  "gene_name": "Kallikrein-14",
  "term_id": "GO:0051604",
  "gene": "UniProtKB:Q9P0G3",
  "term_label": "protein maturation"
}